protein localization to cell division site involved in cell separation after cytokinesis [GO:1904652] (biological process) Definition: Any protein localization to cell division site that is involved in cell separation after cytokinesis. References: PMID:25411334 Sources: GOC:TermGenie, GO_REF:0000060 Relationships: is a type of protein localization to cell division site [GO:0072741]; is part of septum digestion after cytokinesis [GO:0000920]